{
  "gene_name": "Ubiquitin carboxyl-terminal hydrolase 30",
  "term_id": "GO:0004843",
  "gene": "UniProtKB:Q70CQ3",
  "term_label": "cysteine-type deubiquitinase activity",
  "gene_symbol": "USP30"
}